{
  "gene_name": "Dymeclin",
  "term_id": "GO:0007030",
  "term_label": "Golgi organization",
  "gene": "UniProtKB:Q7RTS9",
  "gene_symbol": "DYM"
}